{
  "term_id": "UNKNOWN:0003",
  "gene_name": "POU domain, class 2, transcription factor 2",
  "gene_symbol": "POU2F2",
  "gene": "UniProtKB:P09086",
  "term_label": "Unknown cellular component"
}